{
  "term_id": "UNKNOWN:0002",
  "term_label": "Unknown biological process",
  "gene": "UniProtKB:Q8N402",
  "gene_name": "Putative uncharacterized protein LOC388882",
  "gene_symbol": "Q8N402"
}